{
  "term_label": "Unknown biological process",
  "gene": "UniProtKB:P04278",
  "term_id": "UNKNOWN:0002",
  "gene_name": "Sex hormone-binding globulin",
  "gene_symbol": "SHBG"
}